{
  "gene_name": "E3 ubiquitin-protein ligase RNF167",
  "term_id": "GO:0045786",
  "gene_symbol": "RNF167",
  "gene": "UniProtKB:Q9H6Y7",
  "term_label": "negative regulation of cell cycle"
}